{
  "term_id": "GO:0005634",
  "gene": "UniProtKB:O60224",
  "gene_symbol": "SSX4",
  "term_label": "nucleus",
  "gene_name": "Protein SSX4"
}